{
  "term_id": "GO:0031490",
  "gene": "UniProtKB:A3KN83",
  "gene_name": "Protein strawberry notch homolog 1",
  "gene_symbol": "SBNO1",
  "term_label": "chromatin DNA binding"
}